{
  "term_id": "UNKNOWN:0003",
  "term_label": "Unknown cellular component",
  "gene_name": "Cytochrome P450 3A4",
  "gene_symbol": "CYP3A4",
  "gene": "UniProtKB:P08684"
}